AIM2 inflammasome complex assembly [GO:0140970] (biological process) Regulation: regulated by regulation of AIM2 inflammasome complex assembly [GO:0140971]; negatively regulated by GO:0140972; positively regulated by positive regulation of AIM2 inflammasome complex assembly [GO:0140973] References: PMID:33467177 Relationships: is a type of protein-containing complex assembly [GO:0065003] Definition: The aggregation, arrangement and bonding together of a set of components to form the AIM2 inflammasome complex.